{
  "term_id": "UNKNOWN:0001",
  "gene_symbol": "ECRG4",
  "gene": "UniProtKB:Q9H1Z8",
  "term_label": "Unknown molecular function",
  "gene_name": "Augurin"
}